{
  "gene_symbol": "SLC2A4RG",
  "term_id": "GO:0005634",
  "gene_name": "SLC2A4 regulator",
  "gene": "UniProtKB:Q9NR83",
  "term_label": "nucleus"
}